high-affinity sulfate transmembrane transporter activity [GO:0015381] (molecular function) Sources: GOC:mtg_transport Definition: Enables the secondary active high affinity transfer of sulfate from one side of a membrane to the other. Secondary active transport is the transfer of a solute across a membrane, up its concentration gradient. The transporter binds the solute and undergoes a series of conformational changes. Transport works equally well in either direction and is driven by a chemiosmotic source of energy. Secondary active transporters include symporters and antiporters. In high-affinity transport the transporter is able to bind thesolute even if it is only present at very low concentrations. Also known as: high affinity sulfate transmembrane transporter activity, high affinity sulphate permease activity, high affinity sulfate permease activity Relationships: is a type of secondary active sulfate transmembrane transporter activity [GO:0008271]